{
  "term_id": "GO:0005763",
  "gene": "UniProtKB:P51398",
  "gene_name": "Small ribosomal subunit protein mS29",
  "gene_symbol": "DAP3",
  "term_label": "mitochondrial small ribosomal subunit"
}